{
  "gene": "UniProtKB:O60806",
  "gene_name": "T-box transcription factor TBX19",
  "term_id": "GO:0001708",
  "gene_symbol": "TBX19",
  "term_label": "cell fate specification"
}